{
  "term_label": "plasma membrane",
  "gene_name": "Syntaxin-1A",
  "term_id": "GO:0005886",
  "gene": "UniProtKB:Q16623",
  "gene_symbol": "STX1A"
}